positive regulation of natural killer cell mediated cytotoxicity directed against tumor cell target [GO:0002860] (biological process) Definition: Any process that activates or increases the frequency, rate, or extent of natural killer cell mediated cytotoxicity directed against tumor cell target. Also known as: up regulation of natural killer cell mediated cytotoxicity directed against tumor cell target, up-regulation of natural killer cell mediated cytotoxicity directed against tumor cell target, upregulation of natural killer cell mediated cytotoxicity directed against tumor cell target, activation of natural killer cell mediated cytotoxicity directed against tumor cell target, stimulation of natural killer cell mediated cytotoxicity directed against tumor cell target Sources: GOC:add Relationships: is a type of GO:0002857; is a type of GO:0002858; is a type of positive regulation of natural killer cell mediated cytotoxicity [GO:0045954]; positively regulates natural killer cell mediated cytotoxicity directed against tumor cell target [GO:0002420]